{
  "term_label": "positive regulation of cell motility",
  "gene": "UniProtKB:Q9Y6A4",
  "gene_symbol": "CFAP20",
  "gene_name": "Cilia- and flagella-associated protein 20",
  "term_id": "GO:2000147"
}